{
  "term_id": "GO:0033857",
  "gene_symbol": "PPIP5K1",
  "gene": "UniProtKB:Q6PFW1",
  "gene_name": "Inositol hexakisphosphate and diphosphoinositol-pentakisphosphate kinase 1",
  "term_label": "5-diphosphoinositol pentakisphosphate 1-kinase activity"
}